{
  "term_id": "GO:0045087",
  "gene": "UniProtKB:O75179",
  "term_label": "innate immune response",
  "gene_symbol": "ANKRD17",
  "gene_name": "Ankyrin repeat domain-containing protein 17"
}